{
  "gene_name": "Tektin bundle-interacting protein 1",
  "gene_symbol": "TEKTIP1",
  "term_id": "UNKNOWN:0001",
  "gene": "UniProtKB:A6NCJ1",
  "term_label": "Unknown molecular function"
}